{
  "term_id": "GO:0000785",
  "term_label": "chromatin",
  "gene_symbol": "TSPY4",
  "gene": "UniProtKB:P0CV99",
  "gene_name": "Testis-specific Y-encoded protein 4"
}